{
  "gene_symbol": "PHF7",
  "gene_name": "PHD finger protein 7",
  "gene": "UniProtKB:Q9BWX1",
  "term_label": "Unknown molecular function",
  "term_id": "UNKNOWN:0001"
}